{
  "term_label": "Unknown cellular component",
  "gene": "UniProtKB:O14978",
  "gene_symbol": "ZNF263",
  "term_id": "UNKNOWN:0003",
  "gene_name": "Zinc finger protein 263"
}